negative regulation of juvenile hormone catabolic process [GO:0045970] (BP) Sources: GOC:go_curators Relationships: is a type of GO:0045928; is a type of regulation of juvenile hormone catabolic process [GO:0045952]; is a type of negative regulation of lipid catabolic process [GO:0050995]; negatively regulates juvenile hormone catabolic process [GO:0006719] Definition: Any process that stops, prevents, or reduces the frequency, rate or extent of the chemical reactions and pathways resulting in the breakdown of juvenile hormone. Also known as: down regulation of juvenile hormone catabolic process, down-regulation of juvenile hormone catabolic process, downregulation of juvenile hormone catabolic process, negative regulation of juvenile hormone breakdown, negative regulation of juvenile hormone catabolism, negative regulation of juvenile hormone degradation, inhibition of juvenile hormone catabolic process